{
  "gene": "UniProtKB:Q5R387",
  "term_label": "phospholipid binding",
  "gene_name": "Putative inactive group IIC secretory phospholipase A2",
  "gene_symbol": "PLA2G2C",
  "term_id": "GO:0005543"
}